{
  "term_label": "Unknown biological process",
  "gene_name": "Neuroblastoma breakpoint family member 4",
  "gene_symbol": "NBPF4",
  "gene": "UniProtKB:Q96M43",
  "term_id": "UNKNOWN:0002"
}